{
  "gene_symbol": "ALDH1B1",
  "term_label": "aldehyde metabolic process",
  "gene": "UniProtKB:P30837",
  "term_id": "GO:0006081",
  "gene_name": "Aldehyde dehydrogenase X, mitochondrial"
}